{
  "gene": "UniProtKB:Q6P087",
  "gene_name": "Mitochondrial mRNA pseudouridine synthase RPUSD3",
  "term_id": "UNKNOWN:0003",
  "gene_symbol": "RPUSD3",
  "term_label": "Unknown cellular component"
}